trichodiene synthase activity [GO:0045482] (molecular function) Sources: EC:4.2.3.6, RHEA:12052 Relationships: is a type of sesquiterpene synthase activity [GO:0010334] Definition: Catalysis of the reaction: 2-trans,6-trans-farnesyl diphosphate = diphosphate + trichodiene. Also known as: sesquiterpene cyclase activity, trans,trans-farnesyl-diphosphate diphosphate-lyase (cyclizing, trichodiene-forming), trans,trans-farnesyl-diphosphate sesquiterpenoid-lyase activity, trichodiene synthetase activity